{
  "gene_name": "Vacuolar protein sorting-associated protein 41 homolog",
  "gene": "UniProtKB:P49754",
  "term_label": "protein-membrane adaptor activity",
  "term_id": "GO:0043495",
  "gene_symbol": "VPS41"
}